{
  "gene_name": "DNA oxidative demethylase ALKBH2",
  "term_label": "ferrous iron binding",
  "gene_symbol": "ALKBH2",
  "term_id": "GO:0008198",
  "gene": "UniProtKB:Q6NS38"
}